{
  "gene": "UniProtKB:Q9Y6G3",
  "gene_name": "Large ribosomal subunit protein mL42",
  "term_label": "Unknown molecular function",
  "term_id": "UNKNOWN:0001",
  "gene_symbol": "MRPL42"
}